{
  "gene_symbol": "CFHR1",
  "gene": "UniProtKB:Q03591",
  "term_id": "GO:0006956",
  "term_label": "complement activation",
  "gene_name": "Complement factor H-related protein 1"
}